{
  "gene": "UniProtKB:Q9UJ55",
  "term_id": "GO:0005634",
  "term_label": "nucleus",
  "gene_name": "MAGE-like protein 2",
  "gene_symbol": "MAGEL2"
}